{
  "term_id": "GO:0005634",
  "term_label": "nucleus",
  "gene_symbol": "NR1D1",
  "gene_name": "Nuclear receptor subfamily 1 group D member 1",
  "gene": "UniProtKB:P20393"
}